viral genome integration into host DNA [GO:0044826] (biological process) Definition: The insertion into a host genome of viral DNA, usually by the action of an integrase enzyme. Once integrated, the provirus persists in the host cell and serves as a template for the transcription of viral genes and replication of the viral genome, leading to the production of new viruses. Relationships: is a type of viral process [GO:0016032]; is part of viral life cycle [GO:0019058] References: PMID:19091057 Also known as: viral genome integration